{
  "term_label": "Unknown molecular function",
  "term_id": "UNKNOWN:0001",
  "gene_name": "Superkiller complex protein 3",
  "gene": "UniProtKB:Q6PGP7",
  "gene_symbol": "SKIC3"
}